{
  "gene_name": "Fibroblast growth factor 16",
  "gene": "UniProtKB:O43320",
  "term_id": "GO:0005737",
  "gene_symbol": "FGF16",
  "term_label": "cytoplasm"
}